glycoprotein catabolic process [GO:0006516] (biological process) Also known as: glycoprotein breakdown, glycoprotein catabolism, glycoprotein degradation Definition: The chemical reactions and pathways resulting in the breakdown of a glycoprotein, a protein that contains covalently bound glycose (i.e. monosaccharide) residues; the glycose occurs most commonly as oligosaccharide or fairly small polysaccharide but occasionally as monosaccharide. Relationships: is a type of GO:0009100; is a type of protein catabolic process [GO:0030163]; is a type of carbohydrate derivative catabolic process [GO:1901136] Sources: GOC:go_curators, ISBN:0198506732 Subtypes: GO:0030167, O-sialoglycoprotein catabolic process [GO:0045173], GO:0060309, ubiquitin-dependent glycoprotein ERAD pathway [GO:0097466]